{
  "gene": "UniProtKB:Q9GZY6",
  "term_label": "B cell receptor signaling pathway",
  "gene_name": "Linker for activation of T-cells family member 2",
  "term_id": "GO:0050853",
  "gene_symbol": "LAT2"
}